2-oxoglutarate, L-arginine oxygenase (succinate-forming) activity [GO:0102525] (molecular function) Definition: Catalysis of the reaction: L-argininium(1+) + 2-oxoglutarate + O2 = (3S)-3-hydroxy-L-arginine(1+) + succinate + carbon dioxide. Sources: GOC:pz, RHEA:36607 Relationships: is a type of 2-oxoglutarate-dependent dioxygenase activity [GO:0016706]